{
  "term_label": "nucleus",
  "gene": "UniProtKB:Q9HC44",
  "gene_symbol": "GPBP1L1",
  "gene_name": "Vasculin-like protein 1",
  "term_id": "GO:0005634"
}